{
  "term_label": "ASAP complex",
  "gene_symbol": "ACIN1",
  "term_id": "GO:0061574",
  "gene": "UniProtKB:Q9UKV3",
  "gene_name": "Apoptotic chromatin condensation inducer in the nucleus"
}